{
  "gene_symbol": "TEX19",
  "gene_name": "Testis-expressed protein 19",
  "gene": "UniProtKB:Q8NA77",
  "term_label": "male gonad development",
  "term_id": "GO:0008584"
}